{
  "gene_name": "Tubulin beta-8 chain",
  "gene": "UniProtKB:Q3ZCM7",
  "term_label": "structural constituent of cytoskeleton",
  "gene_symbol": "TUBB8",
  "term_id": "GO:0005200"
}